{
  "term_id": "GO:0001836",
  "gene": "UniProtKB:Q92843",
  "gene_symbol": "BCL2L2",
  "gene_name": "Bcl-2-like protein 2",
  "term_label": "release of cytochrome c from mitochondria"
}